A3 adenosine receptor binding [GO:0031689] (molecular function) Sources: GOC:mah, GOC:nln Also known as: A3 adenosine receptor ligand Definition: Binding to an A3 adenosine receptor. Relationships: is a type of adenosine receptor binding [GO:0031685]